{
  "gene_symbol": "ZNF556",
  "gene": "UniProtKB:Q9HAH1",
  "gene_name": "Zinc finger protein 556",
  "term_id": "GO:0000981",
  "term_label": "DNA-binding transcription factor activity, RNA polymerase II-specific"
}